cellular homeostasis [GO:0019725] (biological process) Relationships: is a type of homeostatic process [GO:0042592] Definition: Any process involved in the maintenance of an internal steady state at the level of the cell. Sources: GOC:isa_complete, GOC:jl, ISBN:0395825172 Subtypes: GO:0006884, GO:0006973, GO:0010992, GO:0045454, muscle cell cellular homeostasis [GO:0046716], GO:0055082, GO:0070050, recycling of RNA polymerase [GO:0140182]